{
  "gene_name": "Aconitate hydratase, mitochondrial",
  "gene": "UniProtKB:Q99798",
  "term_id": "GO:0006099",
  "gene_symbol": "ACO2",
  "term_label": "tricarboxylic acid cycle"
}